glyoxal oxidase activity [GO:0046569] (MF) Definition: Catalysis of the reaction: glyoxal + O2 + H2O = glyoxalate + H2O2. References: PMID:11733005 Also known as: GLOX Relationships: is a type of oxidoreductase activity, acting on the aldehyde or oxo group of donors, oxygen as acceptor [GO:0016623]